{
  "gene": "UniProtKB:Q2M389",
  "term_label": "Unknown molecular function",
  "term_id": "UNKNOWN:0001",
  "gene_name": "WASH complex subunit 4",
  "gene_symbol": "WASHC4"
}